{
  "gene": "UniProtKB:Q9NV88",
  "term_label": "integrator complex",
  "gene_symbol": "INTS9",
  "gene_name": "Integrator complex subunit 9",
  "term_id": "GO:0032039"
}